{
  "gene_name": "DDB1- and CUL4-associated factor 8-like protein 1",
  "gene_symbol": "DCAF8L1",
  "gene": "UniProtKB:A6NGE4",
  "term_label": "Cul4-RING E3 ubiquitin ligase complex",
  "term_id": "GO:0080008"
}